{
  "gene": "UniProtKB:P57073",
  "term_label": "neural crest cell development",
  "term_id": "GO:0014032",
  "gene_symbol": "SOX8",
  "gene_name": "Transcription factor SOX-8"
}